{
  "gene": "UniProtKB:Q969T4",
  "gene_symbol": "UBE2E3",
  "term_id": "GO:0061631",
  "gene_name": "Ubiquitin-conjugating enzyme E2 E3",
  "term_label": "ubiquitin conjugating enzyme activity"
}